{
  "term_label": "Unknown molecular function",
  "gene": "UniProtKB:O75074",
  "term_id": "UNKNOWN:0001",
  "gene_symbol": "LRP3",
  "gene_name": "Low-density lipoprotein receptor-related protein 3"
}